{
  "gene_name": "Anaphase-promoting complex subunit 16",
  "term_label": "anaphase-promoting complex",
  "term_id": "GO:0005680",
  "gene_symbol": "ANAPC16",
  "gene": "UniProtKB:Q96DE5"
}